{
  "gene_symbol": "PLK2",
  "term_label": "mitotic spindle organization",
  "term_id": "GO:0007052",
  "gene_name": "Serine_threonine-protein kinase PLK2",
  "gene": "UniProtKB:Q9NYY3"
}